{
  "gene_symbol": "RCL1",
  "gene": "UniProtKB:Q9Y2P8",
  "term_label": "endonucleolytic cleavage of tricistronic rRNA transcript (SSU-rRNA, 5.8S rRNA, LSU-rRNA)",
  "term_id": "GO:0000479",
  "gene_name": "RNA 3'-terminal phosphate cyclase-like protein"
}